{
  "term_id": "UNKNOWN:0001",
  "gene_symbol": "SPATA18",
  "gene_name": "Mitochondria-eating protein",
  "gene": "UniProtKB:Q8TC71",
  "term_label": "Unknown molecular function"
}